{
  "term_label": "Unknown biological process",
  "gene": "UniProtKB:A0A0U1RQB9",
  "term_id": "UNKNOWN:0002",
  "gene_symbol": "IGHD5-12",
  "gene_name": "Immunoglobulin heavy diversity 5-12 (Fragment)"
}